co-SMAD binding [GO:0070410] (molecular function) Relationships: is a type of SMAD binding [GO:0046332] Definition: Binding to a common mediator SMAD signaling protein. Also known as: common mediator SMAD binding, common partner SMAD binding, common-mediator SMAD binding, common-partner SMAD binding References: PMID:19114992 Sources: GOC:BHF, GOC:vk